{
  "gene": "UniProtKB:Q05397",
  "gene_name": "Focal adhesion kinase 1",
  "term_id": "GO:0005886",
  "gene_symbol": "PTK2",
  "term_label": "plasma membrane"
}